cellular hyperosmotic response [GO:0071474] (biological process) Definition: Any process that results in a change in state or activity of a cell (in terms of movement, secretion, enzyme production, gene expression, etc.) as a result of detection of, or exposure to, a hyperosmotic environment, i.e. an environment with a higher concentration of solutes than the organism or cell. Subtypes: GO:0071475 Also known as: cellular HOG response, cellular hypertonic response, cellular response to hypertonicity Sources: GOC:mah Relationships: is a type of hyperosmotic response [GO:0006972]; is_a cellular response to osmotic stress [GO:0071470]